{
  "gene_symbol": "DNA2",
  "term_label": "RNA binding",
  "term_id": "GO:0003723",
  "gene": "UniProtKB:P51530",
  "gene_name": "DNA replication ATP-dependent helicase_nuclease DNA2"
}